{
  "gene": "UniProtKB:P10124",
  "gene_symbol": "SRGN",
  "term_id": "GO:0030141",
  "term_label": "secretory granule",
  "gene_name": "Serglycin"
}